{
  "term_id": "GO:0043209",
  "gene_name": "Neuronal membrane glycoprotein M6-b",
  "gene": "UniProtKB:Q13491",
  "term_label": "myelin sheath",
  "gene_symbol": "GPM6B"
}